{
  "term_id": "GO:0005550",
  "gene_symbol": "VN1R2",
  "gene": "UniProtKB:Q8NFZ6",
  "gene_name": "Vomeronasal type-1 receptor 2",
  "term_label": "pheromone binding"
}